L-proline catabolic process to L-glutamate [GO:0010133] (biological process) Regulation: regulated by regulation of L-proline catabolic process to L-glutamate [GO:2001156]; RO_0002212 by GO:2001157; RO_0002213 by positive regulation of L-proline catabolic process to L-glutamate [GO:2001158] Sources: MetaCyc:PROUT-PWY Definition: The chemical reactions and pathways resulting in the breakdown of L-proline into L-glutamate. Also known as: proline breakdown to glutamate, proline degradation to glutamate, proline oxidation Relationships: is a type of glutamate metabolic process [GO:0006536]; is a type of L-proline catabolic process [GO:0006562]